negative regulation of glycogen biosynthetic process [GO:0045719] (biological process) Sources: GOC:go_curators Definition: Any process that stops, prevents, or reduces the frequency, rate or extent of the chemical reactions and pathways resulting in the formation of glycogen. Also known as: down regulation of glycogen biosynthetic process, down-regulation of glycogen biosynthetic process, downregulation of glycogen biosynthetic process, negative regulation of glycogen anabolism, negative regulation of glycogen biosynthesis, negative regulation of glycogen formation, negative regulation of glycogen synthesis, inhibition of glycogen biosynthetic process Relationships: is a type of regulation of glycogen biosynthetic process [GO:0005979]; is a type of GO:0010558; is_a GO:0070874; negatively regulates glycogen biosynthetic process [GO:0005978]